maintenance of reproductive diapause [GO:0071984] (biological process) Relationships: is a type of maintenance of diapause [GO:0071982] Definition: The dormancy process that results an organism remaining in reproductive diapause. Reproductive diapause is a form of diapause where the organism itself will remain fully active, including feeding and other routine activities, but the reproductive organs experience a tissue-specific reduction in metabolism, with characteristic triggering and releasing stimuli. Sources: GOC:mah